type 5B serotonin receptor binding [GO:0031831] (molecular function) Definition: Binding to a type 5B serotonin receptor. Relationships: is a type of G protein-coupled serotonin receptor binding [GO:0031821] Also known as: 5-hydroxytryptamine 5B receptor binding, type 5B serotonin receptor ligand Sources: GOC:mah, GOC:nln